kidney morphogenesis [GO:0060993] (biological process) Definition: Morphogenesis of a kidney. A kidney is an organ that filters the blood and excretes the end products of body metabolism in the form of urine. Relationships: is a type of animal organ morphogenesis [GO:0009887]; is part of kidney development [GO:0001822] Subtypes: metanephros morphogenesis [GO:0003338], mesonephros morphogenesis [GO:0061206], pronephros morphogenesis [GO:0072114] Sources: GOC:dph, GOC:mtg_kidney_jan10